B cell apoptotic process [GO:0001783] (biological process) Regulation: regulated by regulation of B cell apoptotic process [GO:0002902]; negatively regulated by negative regulation of B cell apoptotic process [GO:0002903]; positively regulated by GO:0002904 Sources: CL:0000236, GOC:add, GOC:mtg_apoptosis, ISBN:0781735149 Also known as: B cell programmed cell death by apoptosis, B lymphocyte apoptosis, B lymphocyte programmed cell death by apoptosis, B-cell apoptosis, B-cell programmed cell death by apoptosis, B-lymphocyte apoptosis, B-lymphocyte programmed cell death by apoptosis, apoptosis of B cells, apoptosis of B lymphocytes, apoptosis of B-cells, apoptosis of B-lymphocytes, programmed cell death of B cells by apoptosis, programmed cell death of B lymphocytes by apoptosis, programmed cell death of B-cells by apoptosis, programmed cell death of B-lymphocytes by apoptosis, programmed cell death, B cells, programmed cell death, B lymphocytes, programmed cell death, B-cells, programmed cell death, B-lymphocytes, B cell apoptosis Subtypes: B cell deletion [GO:0002516], mature B cell apoptotic process [GO:0002901], activation-induced B cell apoptotic process [GO:0071948] Definition: Any apoptotic process in a B cell, a lymphocyte of B lineage with the phenotype CD19-positive and capable of B cell mediated immunity. Relationships: is a type of lymphocyte apoptotic process [GO:0070227]